hindbrain radial glia guided cell migration [GO:0021932] (biological process) Subtypes: radial glia guided migration of cerebellar granule cell [GO:0021933], radial glia guided migration of Purkinje cell [GO:0021942] Definition: The radially directed movement of a cell along radial glial cells in the hindbrain. Radial migration refers to a directed movement from the internal ventricular area to the outer surface of the hindbrain. References: PMID:15157725 Sources: GOC:cls, GOC:dgh, GOC:dph, GOC:jid, GO_REF:0000021 Relationships: is a type of cell migration in hindbrain [GO:0021535]